{
  "term_id": "GO:0000977",
  "term_label": "RNA polymerase II transcription regulatory region sequence-specific DNA binding",
  "gene": "UniProtKB:P17023",
  "gene_name": "Zinc finger protein 19",
  "gene_symbol": "ZNF19"
}